substrate-independent telencephalic tangential interneuron migration [GO:0021843] (biological process) Subtypes: interneuron migration from the subpallium to the cortex [GO:0021830], GO:0021831 References: PMID:12626695 Sources: GOC:cls, GOC:dgh, GOC:dph, GOC:jid, GO_REF:0000021 Relationships: is a type of substrate-independent telencephalic tangential migration [GO:0021826] Definition: The directional movement of tangentially migrating interneurons that are not guided by attaching to extracellular substrates.